{
  "gene_symbol": "ERCC5",
  "term_label": "nucleus",
  "term_id": "GO:0005634",
  "gene": "UniProtKB:P28715",
  "gene_name": "DNA excision repair protein ERCC-5"
}